{
  "gene_name": "C2 domain-containing protein 3",
  "gene": "UniProtKB:Q4AC94",
  "term_label": "centriolar satellite",
  "gene_symbol": "C2CD3",
  "term_id": "GO:0034451"
}